{
  "gene_symbol": "CEACAM3",
  "term_id": "GO:1990782",
  "gene_name": "Carcinoembryonic antigen-related cell adhesion molecule 3",
  "gene": "UniProtKB:P40198",
  "term_label": "protein tyrosine kinase binding"
}